{
  "term_id": "GO:0006955",
  "gene": "UniProtKB:P15812",
  "gene_symbol": "CD1E",
  "gene_name": "T-cell surface glycoprotein CD1e, membrane-associated",
  "term_label": "immune response"
}